{
  "gene": "UniProtKB:Q7Z4N2",
  "term_id": "GO:0005262",
  "term_label": "calcium channel activity",
  "gene_symbol": "TRPM1",
  "gene_name": "Transient receptor potential cation channel subfamily M member 1"
}